regulation of uterine smooth muscle contraction [GO:0070472] (biological process) Subtypes: GO:0070473, positive regulation of uterine smooth muscle contraction [GO:0070474] Also known as: regulation of myometrial contraction, regulation of myometrial smooth muscle contraction, regulation of myometrium contraction Definition: Any process that modulates the frequency, rate or extent of uterine smooth muscle contraction. Relationships: is_a GO:0006940; regulates uterine smooth muscle contraction [GO:0070471] Sources: GOC:go_curators